{
  "term_id": "GO:0030198",
  "gene_name": "Collagen alpha-1(XXVII) chain",
  "gene_symbol": "COL27A1",
  "gene": "UniProtKB:Q8IZC6",
  "term_label": "extracellular matrix organization"
}